{
  "gene": "UniProtKB:Q8TB96",
  "term_label": "plasma membrane",
  "term_id": "GO:0005886",
  "gene_symbol": "ITFG1",
  "gene_name": "T-cell immunomodulatory protein"
}